actin filament branch point [GO:0061834] (cellular component) Definition: The part of an actin filament where the structure forks. Relationships: is a type of cellular anatomical structure [GO:0110165]; is part of actin filament [GO:0005884] References: PMID:18256280 Also known as: microfilament branch point